{
  "gene_name": "ADP-ribosylation factor-like protein 5B",
  "gene": "UniProtKB:Q96KC2",
  "gene_symbol": "ARL5B",
  "term_id": "GO:0005737",
  "term_label": "cytoplasm"
}